regulation of T cell cytokine production [GO:0002724] (biological process) Sources: GOC:add Relationships: is a type of regulation of T cell mediated immunity [GO:0002709]; is a type of regulation of cytokine production involved in immune response [GO:0002718]; regulates T cell cytokine production [GO:0002369] Subtypes: negative regulation of T cell cytokine production [GO:0002725], positive regulation of T cell cytokine production [GO:0002726], regulation of T-helper 2 cell cytokine production [GO:2000551], regulation of T-helper 1 cell cytokine production [GO:2000554] Definition: Any process that modulates the frequency, rate, or extent of T cell cytokine production. Also known as: regulation of T lymphocyte cytokine production, regulation of T-cell cytokine production, regulation of T-lymphocyte cytokine production